heteropolysaccharide binding [GO:0010297] (molecular function) Relationships: is a type of polysaccharide binding [GO:0030247] Definition: Binding to a heteropolysaccharide, a glycan composed of more than one type of monosaccharide residue. References: PMID:16640603 Also known as: heteroglycan binding Subtypes: GO:2001063, galactomannan binding [GO:2001072]